microfilament motor activity [GO:0000146] (molecular function) Definition: A motor activity that generates movement along a microfilament, driven by ATP hydrolysis. Subtypes: minus-end directed microfilament motor activity [GO:0060001], plus-end directed microfilament motor activity [GO:0060002] Relationships: is a type of cytoskeletal motor activity [GO:0003774]; is a type of polypeptide conformation or assembly isomerase activity [GO:0120544]; is a type of GO:0140657 Also known as: actin filament motor activity, actin-activated ATPase activity, actin-dependent ATPase activity, actin-filament motor activity, muscle motor activity, myosin ATPase activity References: PMID:29716949